{
  "term_id": "GO:0050911",
  "gene_symbol": "OR10J6P",
  "gene": "UniProtKB:Q8NGY7",
  "gene_name": "Putative olfactory receptor 10J6",
  "term_label": "detection of chemical stimulus involved in sensory perception of smell"
}